{
  "gene_symbol": "GRIN3A",
  "gene_name": "Glutamate receptor ionotropic, NMDA 3A",
  "term_label": "postsynaptic density membrane",
  "gene": "UniProtKB:Q8TCU5",
  "term_id": "GO:0098839"
}